positive regulation of neurotransmitter transport [GO:0051590] (biological process) Subtypes: positive regulation of neurotransmitter secretion [GO:0001956], GO:0051582 Relationships: is_a GO:0051050; is a type of regulation of neurotransmitter transport [GO:0051588]; positively regulates neurotransmitter transport [GO:0006836] Also known as: up regulation of neurotransmitter transport, up-regulation of neurotransmitter transport, upregulation of neurotransmitter transport, activation of neurotransmitter transport, stimulation of neurotransmitter transport Definition: Any process that activates or increases the frequency, rate or extent of the directed movement of a neurotransmitter into, out of or within a cell, or between cells, by means of some agent such as a transporter or pore. Sources: GOC:ai